{
  "term_id": "GO:0036064",
  "gene": "UniProtKB:A1XBS5",
  "term_label": "ciliary basal body",
  "gene_symbol": "CIBAR1",
  "gene_name": "CBY1-interacting BAR domain-containing protein 1"
}